{
  "gene_name": "Alpha-2A adrenergic receptor",
  "gene": "UniProtKB:P08913",
  "term_label": "plasma membrane",
  "term_id": "GO:0005886",
  "gene_symbol": "ADRA2A"
}